{
  "term_id": "GO:0016251",
  "gene": "UniProtKB:Q12962",
  "gene_name": "Transcription initiation factor TFIID subunit 10",
  "gene_symbol": "TAF10",
  "term_label": "RNA polymerase II general transcription initiation factor activity"
}